{
  "term_id": "GO:0007155",
  "gene_name": "Protocadherin beta-1",
  "gene_symbol": "PCDHB1",
  "gene": "UniProtKB:Q9Y5F3",
  "term_label": "cell adhesion"
}